actin-dependent nuclear migration [GO:1990974] (biological process) Definition: The process whereby the centrosome is held at the cell center while the nucleus moves to the cell rear by actin retrograde flow resulting in the position of the centrosome between the nucleus and the leading edge of the cell. References: PMID:21173262 Sources: GOC:hjd Also known as: actin-dependent nuclear movement Relationships: is a type of nuclear migration [GO:0007097]